{
  "term_label": "ABC-type bile acid transporter activity",
  "term_id": "GO:0015432",
  "gene_name": "Bile salt export pump",
  "gene": "UniProtKB:O95342",
  "gene_symbol": "ABCB11"
}